{
  "gene_symbol": "KAT6A",
  "gene_name": "Histone acetyltransferase KAT6A",
  "term_label": "nucleus",
  "gene": "UniProtKB:Q92794",
  "term_id": "GO:0005634"
}